sesquiterpene metabolic process [GO:0051761] (biological process) Definition: The chemical reactions and pathways involving sesquiterpenes, any of a class of terpenes of the formula C15H24 or a derivative of such a terpene. Subtypes: sesquiterpene biosynthetic process [GO:0051762], sesquiterpene catabolic process [GO:0051763] Also known as: sesquiterpene metabolism Relationships: is a type of terpene metabolic process [GO:0042214] Sources: GOC:ai